{
  "term_label": "pyridoxal phosphate binding",
  "gene_symbol": "PSAT1",
  "gene_name": "Phosphoserine aminotransferase",
  "gene": "UniProtKB:Q9Y617",
  "term_id": "GO:0030170"
}